{
  "term_label": "Unknown biological process",
  "gene": "UniProtKB:Q6P3W6",
  "gene_symbol": "NBPF10",
  "term_id": "UNKNOWN:0002",
  "gene_name": "Neuroblastoma breakpoint family member 10"
}